{
  "term_label": "regulation of BMP signaling pathway",
  "gene_symbol": "FST",
  "gene": "UniProtKB:P19883",
  "gene_name": "Follistatin",
  "term_id": "GO:0030510"
}